{
  "term_label": "lipid homeostasis",
  "gene_name": "(Lyso)-N-acylphosphatidylethanolamine lipase",
  "gene": "UniProtKB:Q8TB40",
  "gene_symbol": "ABHD4",
  "term_id": "GO:0055088"
}